neutrophil migration [GO:1990266] (BP) Subtypes: neutrophil chemotaxis [GO:0030593], neutrophil extravasation [GO:0072672], neutrophil dispersal [GO:0140635] Regulation: regulated by regulation of neutrophil migration [GO:1902622]; negatively regulated by GO:1902623; positively regulated by positive regulation of neutrophil migration [GO:1902624] Definition: The movement of a neutrophil within or between different tissues and organs of the body. References: PMID:1826836 Relationships: is a type of GO:0097530